purine imidazole-ring cyclase activity [GO:0050230] (molecular function) Sources: EC:4.3.2.4, MetaCyc:PURINE-IMIDAZOLE-RING-CYCLASE-RXN Also known as: DNA-4,6-diamino-5-formamidopyrimidine 8-C,9-N-lyase (cyclizing), DNA-4,6-diamino-5-formamidopyrimidine 8-C,9-N-lyase (cyclizing; DNA-adenine-forming), DNA-4,6-diamino-5-formamidopyrimidine C8-N9-lyase (cyclizing; DNA-adenine-forming) Relationships: is a type of cyclase activity [GO:0009975]; is a type of amidine-lyase activity [GO:0016842] Definition: Catalysis of the reaction: DNA 4,6-diamino-5-formamidopyrimidine = DNA adenine + H2O.